negative regulation of cell proliferation in midbrain [GO:1904934] (biological process) Definition: Any process that stops, prevents or reduces the frequency, rate or extent of cell proliferation in midbrain. References: PMID:18953410, PMID:24431302 Sources: GOC:PARL, GOC:TermGenie, GOC:bf, GO_REF:0000058 Also known as: down regulation of cell proliferation in mesencephalon, down regulation of cell proliferation in midbrain, down-regulation of cell proliferation in mesencephalon, down-regulation of cell proliferation in midbrain, downregulation of cell proliferation in mesencephalon, downregulation of cell proliferation in midbrain, negative regulation of cell proliferation in mesencephalon, inhibition of cell proliferation in mesencephalon, inhibition of cell proliferation in midbrain, down regulation of mesencepahalic cell proliferation, down-regulation of mesencepahalic cell proliferation, downregulation of mesencepahalic cell proliferation, inhibition of mesencepahalic cell proliferation, negative regulation of mesencepahalic cell proliferation Relationships: is a type of GO:1904933; is a type of negative regulation of neural precursor cell proliferation [GO:2000178]; negatively regulates cell proliferation in midbrain [GO:0033278]